G protein-coupled receptor signaling pathway, coupled to cyclic nucleotide second messenger [GO:0007187] (biological process) Relationships: is a type of G protein-coupled receptor signaling pathway [GO:0007186] Sources: GOC:mah, GOC:signaling, ISBN:0815316194 Also known as: G protein signaling, coupled to cyclic nucleotide second messenger, G protein signalling, coupled to cyclic nucleotide second messenger, G-protein coupled receptor signaling pathway, coupled to cyclic nucleotide second messenger, G-protein signaling, coupled to cyclic nucleotide second messenger, G-protein signalling, coupled to cyclic nucleotide second messenger, GPCR signaling pathway via cyclic nucleotide second messenger Definition: A G protein-coupled receptor signaling pathway in which the signal is transmitted via the activation or inhibition of a nucleotide cyclase activity and a subsequent change in the concentration of a cyclic nucleotide. Subtypes: GO:0007199